{
  "term_label": "Unknown molecular function",
  "term_id": "UNKNOWN:0001",
  "gene_name": "Intraflagellar transport protein 140 homolog",
  "gene": "UniProtKB:Q96RY7",
  "gene_symbol": "IFT140"
}